{
  "gene": "UniProtKB:Q9H6A0",
  "gene_symbol": "DENND2D",
  "term_label": "cytosol",
  "term_id": "GO:0005829",
  "gene_name": "DENN domain-containing protein 2D"
}